{
  "term_label": "Unknown molecular function",
  "term_id": "UNKNOWN:0001",
  "gene_symbol": "FAM136A",
  "gene_name": "Protein FAM136A",
  "gene": "UniProtKB:Q96C01"
}